{
  "gene": "UniProtKB:P63267",
  "term_label": "structural constituent of cytoskeleton",
  "gene_name": "Actin, gamma-enteric smooth muscle",
  "term_id": "GO:0005200",
  "gene_symbol": "ACTG2"
}